{
  "gene": "UniProtKB:Q9UPV9",
  "gene_symbol": "TRAK1",
  "term_label": "dendrite",
  "gene_name": "Trafficking kinesin-binding protein 1",
  "term_id": "GO:0030425"
}